cellular response to ATP [GO:0071318] (BP) Sources: GOC:mah Also known as: cellular response to adenosine 5'-triphosphate, cellular response to adenosine triphosphate Subtypes: extracellular ATP signaling [GO:0106167] Definition: Any process that results in a change in state or activity of a cell (in terms of movement, secretion, enzyme production, gene expression, etc.) as a result of an ATP (adenosine 5'-triphosphate) stimulus. Relationships: is a type of response to ATP [GO:0033198]; is a type of GO:1901699; is a type of GO:1901701